regulation of mitotic spindle assembly [GO:1901673] (biological process) Also known as: regulation of spindle assembly involved in mitosis Relationships: is a type of regulation of mitotic spindle organization [GO:0060236]; is a type of regulation of spindle assembly [GO:0090169]; regulates GO:0090307 Definition: Any process that modulates the frequency, rate or extent of mitotic spindle assembly. Subtypes: regulation of mitotic spindle formation (spindle phase one) [GO:0110159] Sources: GOC:TermGenie